{
  "gene": "UniProtKB:O00115",
  "gene_name": "Deoxyribonuclease-2-alpha",
  "term_id": "GO:0006309",
  "term_label": "apoptotic DNA fragmentation",
  "gene_symbol": "DNASE2"
}